transcription-coupled nucleotide-excision repair, DNA damage recognition complex [GO:1990250] (cellular component) Relationships: is a type of nucleotide-excision repair, DNA damage recognition complex [GO:1990249] References: PMID:22331906 Sources: GOC:bhm Definition: A protein complex that is capable of identifying lesions in DNA on the actively transcribed strand of the DNA duplex as well as a small subset of lesions not recognized by the general nucleotide-excision repair pathway. The wide range of substrate specificity suggests that the repair complex recognizes distortions in the DNA helix. It subsequently recruits a nucleotide-excision repair, preincision complex.